{
  "gene_name": "E3 ubiquitin-protein ligase HECW2",
  "gene": "UniProtKB:Q9P2P5",
  "gene_symbol": "HECW2",
  "term_label": "regulation of dendrite morphogenesis",
  "term_id": "GO:0048814"
}